{
  "term_label": "maturation of SSU-rRNA from tricistronic rRNA transcript (SSU-rRNA, 5.8S rRNA, LSU-rRNA)",
  "gene_name": "HEAT repeat-containing protein 1",
  "gene_symbol": "HEATR1",
  "gene": "UniProtKB:Q9H583",
  "term_id": "GO:0000462"
}